{
  "gene_name": "Hydrocephalus-inducing protein homolog",
  "gene_symbol": "HYDIN",
  "gene": "UniProtKB:Q4G0P3",
  "term_label": "cilium movement",
  "term_id": "GO:0003341"
}